{
  "term_id": "GO:0006580",
  "term_label": "ethanolamine metabolic process",
  "gene_symbol": "GDE1",
  "gene_name": "Glycerophosphodiester phosphodiesterase 1",
  "gene": "UniProtKB:Q9NZC3"
}